{
  "gene_symbol": "PXN",
  "gene_name": "Paxillin",
  "gene": "UniProtKB:P49023",
  "term_id": "GO:0043542",
  "term_label": "endothelial cell migration"
}